pyoverdine biosynthetic process [GO:0002049] (BP) Relationships: is a type of siderophore biosynthetic process [GO:0019290]; is a type of GO:0043604 References: PMID:15317763 Definition: The chemical reactions and pathways resulting in the formation of the siderochrome pyoverdine.